polyphenic determination [GO:0048647] (biological process) Sources: GOC:jid Definition: The process in which individuals that have the potential to develop any of several possible distinct developmental paths have their individual developmental fates determined in response to environmental and/or genetic cues. Relationships: is a type of multicellular organismal process [GO:0032501]; is part of multicellular organism development [GO:0007275] Subtypes: caste determination [GO:0048648], GO:0048651, polyphenic determination, influence by genetic factors [GO:0048652]